{
  "gene_symbol": "DELE1",
  "term_label": "mitochondrion",
  "gene_name": "DAP3-binding cell death enhancer 1",
  "term_id": "GO:0005739",
  "gene": "UniProtKB:Q14154"
}